intrahepatic bile duct development [GO:0035622] (biological process) Definition: The progression of the intrahepatic bile ducts over time, from their formation to the mature structure. Intrahepatic bile ducts (bile ducts within the liver) collect bile from bile canaliculi in the liver, and connect to the extrahepatic bile ducts (bile ducts outside the liver). References: PMID:20614624 Sources: GOC:bf Also known as: IHBD development, intrahepatic biliary duct development Relationships: is a type of common bile duct development [GO:0061009]; BFO_0000050 liver development [GO:0001889]